D-glutamate oxidase activity [GO:0047821] (MF) Sources: RHEA:10028 Definition: Catalysis of the reaction: D-glutamate + H2O + O2 = 2-oxoglutarate + H2O2 + NH4+. Also known as: D-glutamate:oxygen oxidoreductase (deaminating), D-glutamic acid oxidase activity, D-glutamic oxidase activity Relationships: is a type of D-amino-acid oxidase activity [GO:0003884]